{
  "gene": "UniProtKB:P48163",
  "gene_name": "NADP-dependent malic enzyme",
  "term_id": "GO:0004473",
  "term_label": "malate dehydrogenase (decarboxylating) (NADP+) activity",
  "gene_symbol": "ME1"
}